{
  "term_label": "histone reader activity",
  "gene_name": "Peregrin",
  "term_id": "GO:0140566",
  "gene_symbol": "BRPF1",
  "gene": "UniProtKB:P55201"
}